glycine metabolic process [GO:0006544] (biological process) Subtypes: glycine biosynthetic process [GO:0006545], glycine catabolic process [GO:0006546], glycine betaine biosynthetic process from glycine [GO:0019286], GO:0019352, tetrapyrrole biosynthetic process from glycine and succinyl-CoA [GO:0033527] Sources: GOC:go_curators Also known as: glycine metabolism Relationships: is a type of proteinogenic amino acid metabolic process [GO:0170039]; is a type of alpha-amino acid metabolic process [GO:1901605] Definition: The chemical reactions and pathways involving glycine, aminoethanoic acid.